{
  "gene_symbol": "RAB24",
  "gene": "UniProtKB:Q969Q5",
  "term_label": "intracellular protein transport",
  "term_id": "GO:0006886",
  "gene_name": "Ras-related protein Rab-24"
}